{
  "gene_symbol": "CHMP2B",
  "gene": "UniProtKB:Q9UQN3",
  "term_id": "GO:0005771",
  "term_label": "multivesicular body",
  "gene_name": "Charged multivesicular body protein 2b"
}